signal complex assembly [GO:0007172] (biological process) Definition: The aggregation, arrangement and bonding together of a set of components to form a complex capable of relaying a signal within a cell. Relationships: is a type of regulation of signal transduction [GO:0009966]; is a type of protein-containing complex assembly [GO:0065003] References: PMID:9646862 Sources: GOC:bf, GOC:signaling Also known as: signal complex formation